{
  "gene": "UniProtKB:Q96C34",
  "term_id": "UNKNOWN:0001",
  "term_label": "Unknown molecular function",
  "gene_name": "RUN domain-containing protein 1",
  "gene_symbol": "RUNDC1"
}